development of secondary female sexual characteristics [GO:0046543] (biological process) Definition: The process whose specific outcome is the progression of the secondary female sexual characteristics over time, from their formation to the mature structures. In female humans, these include growth of axillary and pubic hair, breast development and menstrual periods. Their development occurs in response to sex hormone secretion. Sources: GOC:ai Relationships: is a type of development of secondary sexual characteristics [GO:0045136] Subtypes: GO:0042695